negative regulation of telomere maintenance via recombination [GO:0032208] (biological process) Definition: Any process that stops, prevents, or reduces the frequency, rate or extent of a recombinational process involved in the maintenance of proper telomeric length. Sources: GOC:mah Also known as: down regulation of telomere maintenance via recombination, down-regulation of telomere maintenance via recombination, downregulation of telomere maintenance via recombination, inhibition of telomere maintenance via recombination Relationships: is a type of GO:0032205; is a type of regulation of telomere maintenance via recombination [GO:0032207]; is a type of GO:0045950; is_a negative regulation of DNA recombination at telomere [GO:0048239]; negatively regulates telomere maintenance via recombination [GO:0000722]